{
  "gene_symbol": "CNDP2",
  "term_id": "GO:0006508",
  "term_label": "proteolysis",
  "gene": "UniProtKB:Q96KP4",
  "gene_name": "Cytosolic non-specific dipeptidase"
}